{
  "gene": "UniProtKB:Q8N7C3",
  "gene_symbol": "TRIML2",
  "gene_name": "Probable E3 ubiquitin-protein ligase TRIML2",
  "term_label": "innate immune response",
  "term_id": "GO:0045087"
}